{
  "gene_name": "Sterile alpha motif domain-containing protein 15",
  "term_id": "GO:0007165",
  "term_label": "signal transduction",
  "gene": "UniProtKB:Q9P1V8",
  "gene_symbol": "SAMD15"
}